peptide chain release factor N(5)-glutamine methyltransferase activity [GO:0102559] (molecular function) Definition: Catalysis of the reaction: L-glutaminyl-[peptide chain release factor] + S-adenosyl-L-methionine = N(5)-methyl-L-glutaminyl-[peptide chain release factor] + S-adenosyl-L-homocysteine + H+. Sources: RHEA:42896 Also known as: protein-(glutamine-N5) methyltransferase activity Relationships: is a type of GO:0036009